{
  "gene_symbol": "P2RX4",
  "term_label": "calcium ion transmembrane transport",
  "gene": "UniProtKB:Q99571",
  "gene_name": "P2X purinoceptor 4",
  "term_id": "GO:0070588"
}